{
  "gene_symbol": "MED14",
  "term_label": "mediator complex",
  "gene_name": "Mediator of RNA polymerase II transcription subunit 14",
  "term_id": "GO:0016592",
  "gene": "UniProtKB:O60244"
}